amino acid transmembrane import into vacuole [GO:0032975] (biological process) Definition: The directed movement of amino acids into the vacuole across the vacuolar membrane. Sources: GOC:mah Also known as: vacuolar amino acid import Relationships: is a type of GO:0003333; is a type of vacuolar transmembrane transport [GO:0034486] Subtypes: GO:0034490, neutral amino acid transmembrane import into vacuole [GO:0034491], glutamate transmembrane import into vacuole [GO:0090454], L-tyrosine transmembrane import into vacuole [GO:0090514], GO:1990591